dense core granule docking [GO:0061790] (biological process) Definition: The initial attachment of a dense core granule membrane to the plasma membrane. References: PMID:26575293 Sources: GOC:PARL, GOC:bf Relationships: is a type of vesicle docking involved in exocytosis [GO:0006904]; is part of dense core granule exocytosis [GO:1990504]